{
  "term_id": "GO:0034362",
  "gene": "UniProtKB:P02649",
  "gene_name": "Apolipoprotein E",
  "term_label": "low-density lipoprotein particle",
  "gene_symbol": "APOE"
}